{
  "term_label": "P-body",
  "term_id": "GO:0000932",
  "gene_name": "DNA dC-dU-editing enzyme APOBEC-3A",
  "gene": "UniProtKB:P31941",
  "gene_symbol": "APOBEC3A"
}